{
  "gene": "UniProtKB:P02654",
  "term_label": "negative regulation of lipid catabolic process",
  "gene_symbol": "APOC1",
  "term_id": "GO:0050995",
  "gene_name": "Apolipoprotein C-I"
}